{
  "term_label": "Unknown molecular function",
  "gene_name": "Keratin-associated protein 19-1",
  "gene_symbol": "KRTAP19-1",
  "gene": "UniProtKB:Q8IUB9",
  "term_id": "UNKNOWN:0001"
}